dGMP metabolic process [GO:0046054] (biological process) Relationships: is a type of purine deoxyribonucleotide metabolic process [GO:0009151]; is_a GO:0009170 Also known as: dGMP metabolism Subtypes: dGMP biosynthetic process [GO:0006181], dGMP catabolic process [GO:0046055] Definition: The chemical reactions and pathways involving dGMP, deoxyguanosine monophosphate (2'-deoxyguanosine 5'-phosphate). Sources: GOC:go_curators